{
  "gene_symbol": "ARHGAP31",
  "term_id": "GO:0030027",
  "gene_name": "Rho GTPase-activating protein 31",
  "term_label": "lamellipodium",
  "gene": "UniProtKB:Q2M1Z3"
}